fruit ripening [GO:0009835] (biological process) Definition: An developmental maturation process that has as participant a fruit. Ripening causes changes in one or more characteristics of a fruit (color, aroma, flavor, texture, hardness, cell wall structure) and may make it more attractive to animals and aid in seed dispersal. Relationships: is a type of anatomical structure maturation [GO:0071695]; is part of fruit development [GO:0010154] Sources: GOC:lr Subtypes: fruit ripening, climacteric [GO:0009836], fruit ripening, non-climacteric [GO:0009837] Also known as: fruit maturation, fruit senescence